{
  "gene_name": "PHD finger protein 13",
  "term_id": "GO:0007076",
  "term_label": "mitotic chromosome condensation",
  "gene_symbol": "PHF13",
  "gene": "UniProtKB:Q86YI8"
}